{
  "gene": "UniProtKB:Q9UBD6",
  "term_id": "GO:0097272",
  "gene_symbol": "RHCG",
  "gene_name": "Ammonium transporter Rh type C",
  "term_label": "ammonium homeostasis"
}